{
  "term_id": "GO:0010008",
  "gene_name": "DnaJ homolog subfamily C member 13",
  "gene": "UniProtKB:O75165",
  "gene_symbol": "DNAJC13",
  "term_label": "endosome membrane"
}